P-type potassium:proton transporter activity [GO:0008900] (molecular function) Also known as: proton pump activity, hydrogen/potassium-exchanging ATPase activity, hydrogen:potassium exchanging ATPase activity, hydrogen:potassium-exchanging ATPase activity, gastric H+/K(+) ATPase activity, gastric H+/K+ ATPase, (K+ + H+)-ATPase activity, ATP phosphohydrolase (H+/K+-exchanging), H+-K+-ATPase activity, H+/K(+)-ATPase activity, H+/K(+)-exchanging ATPase activity, H+/K+-ATPase activity, H+/K+-exchanging ATPase activity, H,K-ATPase activity, potassium:proton exchanging ATPase activity Sources: RHEA:22044 Regulation: regulated by regulation of potassium:proton exchanging ATPase activity [GO:1904451] Definition: Enables the transfer of a solute or solutes from one side of a membrane to the other according to the reaction: ATP + H2O + H+(in) + K+(out) = ADP + phosphate + H+(out) + K+(in). Relationships: is a type of P-type proton-exporting transporter activity [GO:0008553]; is a type of GO:0008556